{
  "gene_symbol": "CHMP4A",
  "term_label": "nuclear membrane reassembly",
  "gene": "UniProtKB:Q9BY43",
  "term_id": "GO:0031468",
  "gene_name": "Charged multivesicular body protein 4a"
}